H1 histamine receptor binding [GO:0031807] (molecular function) Definition: Binding to a H1 histamine receptor. Sources: GOC:mah, GOC:nln Also known as: H1 histamine receptor ligand Relationships: is a type of G protein-coupled histamine receptor binding [GO:0031806]